{
  "gene": "UniProtKB:Q01469",
  "gene_symbol": "FABP5",
  "term_label": "nucleus",
  "term_id": "GO:0005634",
  "gene_name": "Fatty acid-binding protein 5"
}